{
  "gene_symbol": "NRIP1",
  "term_id": "GO:0003713",
  "gene": "UniProtKB:P48552",
  "term_label": "transcription coactivator activity",
  "gene_name": "Nuclear receptor-interacting protein 1"
}